{
  "gene": "UniProtKB:Q16658",
  "gene_name": "Fascin",
  "term_label": "growth cone",
  "term_id": "GO:0030426",
  "gene_symbol": "FSCN1"
}